{
  "gene": "UniProtKB:P23610",
  "term_label": "Unknown molecular function",
  "gene_symbol": "F8A3",
  "term_id": "UNKNOWN:0001",
  "gene_name": "40-kDa huntingtin-associated protein"
}